gene expression [GO:0010467] (biological process) References: PMID:25934543, PMID:31580950 Sources: GOC:txnOH-2018 Definition: The process in which a gene's sequence is converted into a mature gene product (protein or RNA). This includes the production of an RNA transcript and its processing, as well as translation and maturation for protein-coding genes. Relationships: is a type of macromolecule biosynthetic process [GO:0009059] Subtypes: cytokine production [GO:0001816], production of molecular mediator of immune response [GO:0002440], oxytocin production [GO:0036162], mitochondrial gene expression [GO:0140053], plastid gene expression [GO:0140899], GO:1901148 Regulation: regulated by regulation of gene expression [GO:0010468]; positively regulated by GO:0010628; negatively regulated by negative regulation of gene expression [GO:0010629]